{
  "gene_name": "Inactive serine protease 54",
  "gene": "UniProtKB:Q6PEW0",
  "gene_symbol": "PRSS54",
  "term_id": "GO:0005615",
  "term_label": "extracellular space"
}